{
  "term_id": "GO:0005886",
  "gene": "UniProtKB:Q9UGM1",
  "gene_name": "Neuronal acetylcholine receptor subunit alpha-9",
  "gene_symbol": "CHRNA9",
  "term_label": "plasma membrane"
}